{
  "term_label": "glyceraldehyde-3-phosphate dehydrogenase (NAD+) (phosphorylating) activity",
  "gene_symbol": "GAPDHS",
  "gene": "UniProtKB:O14556",
  "term_id": "GO:0004365",
  "gene_name": "Glyceraldehyde-3-phosphate dehydrogenase, testis-specific"
}